{
  "gene_name": "Seizure protein 6 homolog",
  "term_label": "dendritic spine",
  "term_id": "GO:0043197",
  "gene": "UniProtKB:Q53EL9",
  "gene_symbol": "SEZ6"
}